ionocyte differentiation [GO:0062236] (biological process) Definition: The process in which a relatively unspecialized cell acquires specialized structural and/or functional features of an ionocyte. Ionocytes are specialized epithelial cells that contribute to osmotic homeostasis. Relationships: is a type of epithelial cell differentiation [GO:0030855] References: PMID:17555741